regulation of maltotriulose transport [GO:1900324] (biological process) Definition: Any process that modulates the frequency, rate or extent of maltotriulose transport. Sources: GOC:TermGenie, GOC:mengo_curators Relationships: is_a regulation of transport [GO:0051049]; regulates maltotriulose transport [GO:2001090] Subtypes: negative regulation of maltotriulose transport [GO:1900325], positive regulation of maltotriulose transport [GO:1900326]